{
  "gene": "UniProtKB:P32004",
  "gene_name": "Neural cell adhesion molecule L1",
  "term_id": "GO:0030424",
  "term_label": "axon",
  "gene_symbol": "L1CAM"
}